{
  "gene_name": "Prokineticin receptor 2",
  "term_id": "GO:0032870",
  "gene_symbol": "PROKR2",
  "term_label": "cellular response to hormone stimulus",
  "gene": "UniProtKB:Q8NFJ6"
}